{
  "term_id": "GO:0007411",
  "term_label": "axon guidance",
  "gene": "UniProtKB:Q15078",
  "gene_name": "Cyclin-dependent kinase 5 activator 1",
  "gene_symbol": "CDK5R1"
}